digestive system process [GO:0022600] (biological process) Definition: A physical, chemical, or biochemical process carried out by living organisms to break down ingested nutrients into components that may be easily absorbed and directed into metabolism. Regulation: regulated by regulation of digestive system process [GO:0044058]; positively regulated by GO:0060456; negatively regulated by negative regulation of digestive system process [GO:0060457] Relationships: is a type of system process [GO:0003008]; is part of GO:0007586 Sources: GOC:isa_complete, GOC:jid, GOC:mtg_cardio Subtypes: gastric acid secretion [GO:0001696], pancreatic juice secretion [GO:0030157], maintenance of gastrointestinal epithelium [GO:0030277], GO:0030421, gastric motility [GO:0035482], rumination [GO:0036147], hindgut contraction [GO:0043133], GO:0046541, intestinal absorption [GO:0050892], GO:0071626, intestinal motility [GO:0120054]